{
  "term_label": "Swi5-Sfr1 complex",
  "gene_name": "Swi5-dependent recombination DNA repair protein 1 homolog",
  "gene_symbol": "SFR1",
  "gene": "UniProtKB:Q86XK3",
  "term_id": "GO:0032798"
}